IRE1-RACK1-PP2A complex [GO:1990630] (CC) Also known as: IRE1alpha-RACK1-PP2A complex, ERN1-RACK1-PP2A complex References: PMID:20103773 Sources: GOC:PARL, GOC:bf Relationships: is a type of protein-containing complex [GO:0032991] Definition: A protein complex consisting of IRE1 (Inositol-requiring enzyme-1), RACK1 (Receptor of activated protein kinase C 1, GNB2L1) and PP2A (protein phosphatase 2A). RACK1 acts as an adaptor to bridge an interaction between IRE1 and PP2A.